{
  "term_id": "UNKNOWN:0001",
  "gene_name": "Integral membrane protein GPR180",
  "gene_symbol": "GPR180",
  "gene": "UniProtKB:Q86V85",
  "term_label": "Unknown molecular function"
}